{
  "term_id": "GO:0005783",
  "gene_name": "Protein TUNAR",
  "gene": "UniProtKB:A0A1B0GTB2",
  "gene_symbol": "TUNAR",
  "term_label": "endoplasmic reticulum"
}